{
  "term_id": "GO:0016973",
  "term_label": "poly(A)+ mRNA export from nucleus",
  "gene_name": "Nuclear pore complex protein Nup93",
  "gene_symbol": "NUP93",
  "gene": "UniProtKB:Q8N1F7"
}